{
  "gene_name": "Vesicle-associated membrane protein 7",
  "term_label": "exocytosis",
  "gene_symbol": "VAMP7",
  "gene": "UniProtKB:P51809",
  "term_id": "GO:0006887"
}